{
  "gene": "UniProtKB:Q8IWQ3",
  "gene_symbol": "BRSK2",
  "term_id": "GO:0050321",
  "term_label": "tau-protein kinase activity",
  "gene_name": "Serine_threonine-protein kinase BRSK2"
}